{
  "term_id": "UNKNOWN:0003",
  "gene_name": "Zinc finger protein 676",
  "term_label": "Unknown cellular component",
  "gene_symbol": "ZNF676",
  "gene": "UniProtKB:Q8N7Q3"
}